nucleoside-triphosphatase regulator activity [GO:0060589] (molecular function) Also known as: NTPase regulator activity Relationships: is a type of enzyme regulator activity [GO:0030234]; regulates ribonucleoside triphosphate phosphatase activity [GO:0017111] Definition: Binds to and modulates the activity of an NTPase. Subtypes: GTPase regulator activity [GO:0030695] Sources: GOC:dph, GOC:tb